{
  "term_label": "ATPase inhibitor activity",
  "term_id": "GO:0042030",
  "gene": "UniProtKB:Q8TF40",
  "gene_symbol": "FNIP1",
  "gene_name": "Folliculin-interacting protein 1"
}